{
  "gene_symbol": "TRIM69",
  "term_label": "innate immune response",
  "gene": "UniProtKB:Q86WT6",
  "term_id": "GO:0045087",
  "gene_name": "E3 ubiquitin-protein ligase TRIM69"
}